regulation of endoplasmic reticulum stress-induced neuron intrinsic apoptotic signaling pathway [GO:1903381] (biological process) Sources: GOC:PARL, GOC:TermGenie, GOC:bf, GO_REF:0000058 Definition: Any process that modulates the frequency, rate or extent of an endoplasmic reticulum stress-induced neuron intrinsic apoptotic signaling pathway. Subtypes: negative regulation of endoplasmic reticulum stress-induced neuron intrinsic apoptotic signaling pathway [GO:1903382] Also known as: regulation of ER stress-induced neuron apoptosis, regulation of endoplasmic reticulum stress-induced neuron apoptosis, regulation of ER stress-induced neuron intrinsic apoptotic signaling pathway, regulation of neuron intrinsic apoptotic signaling pathway in response to endoplasmic reticulum stress Relationships: is a type of GO:0043523; is a type of regulation of endoplasmic reticulum stress-induced intrinsic apoptotic signaling pathway [GO:1902235]; regulates neuron intrinsic apoptotic signaling pathway in response to endoplasmic reticulum stress [GO:0036483]